{
  "term_id": "GO:0007155",
  "gene": "UniProtKB:P20138",
  "gene_name": "Myeloid cell surface antigen CD33",
  "gene_symbol": "CD33",
  "term_label": "cell adhesion"
}